hydrazine synthase activity [GO:0140304] (molecular function) Sources: RHEA:49816 Definition: Catalysis of the reaction: hydrazine + 3 Fe(III)-[cytochrome c] + H2O = nitric oxide + 3 Fe(II)-[cytochrome c] + NH4+ + 2 H+. Relationships: is a type of oxidoreductase activity, acting on other nitrogenous compounds as donors, cytochrome as acceptor [GO:0016662]